{
  "term_id": "GO:0140036",
  "gene_name": "Ankyrin repeat domain-containing protein 13A",
  "gene": "UniProtKB:Q8IZ07",
  "gene_symbol": "ANKRD13A",
  "term_label": "ubiquitin-modified protein reader activity"
}